{
  "term_id": "GO:0007186",
  "gene_symbol": "GPR20",
  "gene": "UniProtKB:Q99678",
  "gene_name": "G-protein coupled receptor 20",
  "term_label": "G protein-coupled receptor signaling pathway"
}